{
  "gene": "UniProtKB:P28336",
  "gene_symbol": "NMBR",
  "term_label": "G protein-coupled receptor signaling pathway",
  "gene_name": "Neuromedin-B receptor",
  "term_id": "GO:0007186"
}